{
  "term_id": "UNKNOWN:0001",
  "gene_name": "Putative uncharacterized protein encoded by LINC00471",
  "gene_symbol": "LINC00471",
  "term_label": "Unknown molecular function",
  "gene": "UniProtKB:Q8N535"
}